{
  "term_id": "GO:0005829",
  "gene_symbol": "DNAJB4",
  "term_label": "cytosol",
  "gene": "UniProtKB:Q9UDY4",
  "gene_name": "DnaJ homolog subfamily B member 4"
}